{
  "gene_name": "Transmembrane channel-like protein 8",
  "term_id": "GO:0008381",
  "gene_symbol": "TMC8",
  "gene": "UniProtKB:Q8IU68",
  "term_label": "mechanosensitive monoatomic ion channel activity"
}